mitochondrial respirasome assembly [GO:0097250] (biological process) Also known as: mitochondrial respiratory chain supercomplex assembly, mitochondrial respiratory supercomplex assembly Definition: The aggregation, arrangement and bonding together of respiratory enzyme complexes I, III and IV of the mitochondrial inner membrane to form a large supercomplex. References: PMID:30030361, PMID:32311046 Relationships: is a type of mitochondrion organization [GO:0007005]; is a type of mitochondrial respiratory chain complex assembly [GO:0033108]